{
  "term_label": "mitotic cell cycle",
  "gene": "UniProtKB:P68366",
  "gene_name": "Tubulin alpha-4A chain",
  "term_id": "GO:0000278",
  "gene_symbol": "TUBA4A"
}